{
  "term_label": "oxygen transport",
  "gene_symbol": "NGB",
  "gene_name": "Neuroglobin",
  "gene": "UniProtKB:Q9NPG2",
  "term_id": "GO:0015671"
}